{
  "gene_symbol": "NRXN2",
  "term_id": "GO:0007165",
  "term_label": "signal transduction",
  "gene": "UniProtKB:Q9P2S2",
  "gene_name": "Neurexin-2"
}